stomatogastric nervous system development [GO:0007421] (biological process) Definition: The process whose specific outcome is the progression of the stomatogastric nervous system over time, from its formation to the mature structure. Relationships: is_a system development [GO:0048731]; is part of nervous system development [GO:0007399] Sources: GOC:jid